{
  "term_id": "GO:0006749",
  "gene_name": "Glutathione S-transferase A2",
  "term_label": "glutathione metabolic process",
  "gene": "UniProtKB:P09210",
  "gene_symbol": "GSTA2"
}